semaphorin receptor binding [GO:0030215] (molecular function) Definition: Binding to a semaphorin receptor. References: PMID:12001990 Sources: GOC:ceb Also known as: plexin binding, plexin ligand, semaphorin receptor ligand Relationships: is a type of GO:0005102